cell differentiation [GO:0030154] (biological process) Subtypes: vasculogenesis [GO:0001570], osteoblast differentiation [GO:0001649], GO:0001742, inner cell mass cell differentiation [GO:0001826], GO:0001829, GO:0002062, hematopoietic progenitor cell differentiation [GO:0002244], follicular dendritic cell differentiation [GO:0002268], GO:0002521, GO:0008583, antipodal cell differentiation [GO:0009557], embryo sac central cell differentiation [GO:0009559], GO:0009560, synergid differentiation [GO:0009563], oocyte differentiation [GO:0009994], glial cell differentiation [GO:0010001], trichome differentiation [GO:0010026], ectodermal cell differentiation [GO:0010668], sclerenchyma cell differentiation [GO:0014001], GO:0014016, cell differentiation in spinal cord [GO:0021515], cell differentiation in hindbrain [GO:0021533], hypothalamus cell differentiation [GO:0021979], GO:0022008, GO:0022036, GO:0022619, microgametophyte vegetative cell differentiation [GO:0022620], GO:0030099, GO:0030182, epithelial cell differentiation [GO:0030855], sorocarp stalk cell differentiation [GO:0031149], GO:0033327, cardiocyte differentiation [GO:0035051], skeletal muscle cell differentiation [GO:0035914], endodermal cell differentiation [GO:0035987], tendon cell differentiation [GO:0035990], myofibroblast differentiation [GO:0036446], GO:0042386, compound eye cone cell differentiation [GO:0042675], GO:0042692, GO:0044671, fat cell differentiation [GO:0045444], myoblast differentiation [GO:0045445], pollen sperm cell differentiation [GO:0048235], mesodermal cell differentiation [GO:0048333], spermatid differentiation [GO:0048515], sporocyte differentiation [GO:0048533], anther wall tapetum cell differentiation [GO:0048657], plant parenchymal cell differentiation [GO:0048760], GO:0048761, mesenchymal cell differentiation [GO:0048762], pigment cell precursor differentiation [GO:0048824], GO:0048863, GO:0048888, GO:0048889, GO:0050931, GO:0060034, GO:0060126, prolactin secreting cell differentiation [GO:0060127], corticotropin hormone secreting cell differentiation [GO:0060128], transdifferentiation [GO:0060290], lung cell differentiation [GO:0060479], GO:0060591, cell differentiation involved in salivary gland development [GO:0060689], cell differentiation involved in embryonic placenta development [GO:0060706], chorionic trophoblast cell differentiation [GO:0060718], GO:0061005, renal filtration cell differentiation [GO:0061318], Malpighian tubule tip cell differentiation [GO:0061382], hepatic stellate cell differentiation [GO:0061521], foam cell differentiation [GO:0090077], GO:0090603, plant epidermal cell differentiation [GO:0090627], cell differentiation involved in phenotypic switching [GO:0090679], GO:0160058, GO:1903498, luteal cell differentiation [GO:1903728], pericyte cell differentiation [GO:1904238], tracheary element differentiation [GO:1905177] Relationships: is a type of cellular developmental process [GO:0048869] Definition: The cellular developmental process in which a relatively unspecialized cell, e.g. embryonic or regenerative cell, acquires specialized structural and/or functional features that characterize a specific cell. Differentiation includes the processes involved in commitment of a cell to a specific fate and its subsequent development to the mature state. Regulation: regulated by GO:0045595; negatively regulated by negative regulation of cell differentiation [GO:0045596]; positively regulated by GO:0045597 Sources: ISBN:0198506732